centrosomal core [GO:0140918] (cellular component) References: PMID:28104305, PMID:30413081 Also known as: centrosome core Relationships: is a type of cellular anatomical structure [GO:0110165]; is part of centrosome [GO:0005813] Definition: The core region of the centrosome, a layered structure containing proteins, surrounded by the centrosomal corona. The core duplicates once per cell cycle at the G2/M transition when two outer layers form the mitotic spindle poles.